{
  "gene_name": "Interferon-induced protein 44",
  "gene_symbol": "IFI44",
  "gene": "UniProtKB:Q8TCB0",
  "term_label": "Unknown cellular component",
  "term_id": "UNKNOWN:0003"
}